{
  "term_id": "GO:0004984",
  "gene": "UniProtKB:Q8NH92",
  "gene_symbol": "OR1S1",
  "term_label": "olfactory receptor activity",
  "gene_name": "Olfactory receptor 1S1"
}